{
  "gene_symbol": "INSC",
  "gene_name": "Protein inscuteable homolog",
  "gene": "UniProtKB:Q1MX18",
  "term_label": "regulation of asymmetric cell division",
  "term_id": "GO:0009786"
}